{
  "gene_name": "Baculoviral IAP repeat-containing protein 5",
  "gene": "UniProtKB:O15392",
  "term_label": "mitotic cytokinesis",
  "gene_symbol": "BIRC5",
  "term_id": "GO:0000281"
}